{
  "gene": "UniProtKB:Q96KN2",
  "term_id": "GO:0016805",
  "gene_name": "Beta-Ala-His dipeptidase",
  "term_label": "dipeptidase activity",
  "gene_symbol": "CNDP1"
}